cellular response to tetrahydrofolate [GO:1904482] (biological process) Definition: Any process that results in a change in state or activity of a cell (in terms of movement, secretion, enzyme production, gene expression, etc.) as a result of a tetrahydrofolate stimulus. References: PMID:24698160 Sources: GOC:BHF, GOC:TermGenie, GOC:hal, GO_REF:0000071 Relationships: is a type of cellular response to nitrogen compound [GO:1901699]; is_a cellular response to oxygen-containing compound [GO:1901701]; is a type of response to tetrahydrofolate [GO:1904481]